RAGE receptor binding [GO:0050786] (molecular function) Relationships: is a type of GO:0005102 Definition: Binding to a RAGE receptor, the receptor for advanced glycation end-products. Sources: GOC:ai Also known as: advanced glycation end-product receptor binding